regulation of cell wall (1->3)-alpha-glucan biosynthetic process [GO:0070608] (biological process) Definition: Any process that modulates the frequency, rate or extent of the chemical reactions and pathways resulting in the formation of (1->3)-alpha-D-glucans, compounds composed of glucose residues linked by (1->3)-alpha-D-glucosidic bonds, found in the walls of cells. Subtypes: regulation of fungal-type cell wall (1->3)-alpha-glucan biosynthetic process [GO:0070610] Relationships: is a type of GO:0010981; is a type of GO:0070606; regulates cell wall (1->3)-alpha-glucan biosynthetic process [GO:0070598] Also known as: regulation of cell wall 1,3-alpha-glucan anabolism, regulation of cell wall 1,3-alpha-glucan biosynthesis, regulation of cell wall 1,3-alpha-glucan biosynthetic process, regulation of cell wall 1,3-alpha-glucan formation, regulation of cell wall 1,3-alpha-glucan synthesis, regulation of cell wall alpha-1,3-glucan anabolism, regulation of cell wall alpha-1,3-glucan biosynthesis, regulation of cell wall alpha-1,3-glucan biosynthetic process, regulation of cell wall alpha-1,3-glucan formation, regulation of cell wall alpha-1,3-glucan synthesis Sources: GOC:mah